L-glycol dehydrogenase activity [GO:0050026] (molecular function) Definition: Catalysis of the reaction: an L-glycol + NAD(P)+ = a 2-hydroxycarbonyl compound + NAD(P)H + H+. Relationships: is a type of oxidoreductase activity, acting on the CH-OH group of donors, NAD or NADP as acceptor [GO:0016616] Sources: EC:1.1.1.185, MetaCyc:L-GLYCOL-DEHYDROGENASE-RXN Also known as: L-(+)-glycol:NAD(P) oxidoreductase activity, L-glycol:NAD(P) dehydrogenase activity, L-glycol:NAD(P)+ oxidoreductase activity, glycol (nicotinamide adenine dinucleotide (phosphate)) dehydrogenase activity